{
  "gene_name": "T-cell antigen CD7",
  "gene": "UniProtKB:P09564",
  "term_label": "Unknown cellular component",
  "term_id": "UNKNOWN:0003",
  "gene_symbol": "CD7"
}